{
  "term_label": "Unknown molecular function",
  "gene_name": "Probable G-protein coupled receptor 153",
  "gene": "UniProtKB:Q6NV75",
  "term_id": "UNKNOWN:0001",
  "gene_symbol": "GPR153"
}